{
  "term_label": "calcium ion binding",
  "gene_name": "Protein S100-A4",
  "term_id": "GO:0005509",
  "gene_symbol": "S100A4",
  "gene": "UniProtKB:P26447"
}